{
  "gene": "UniProtKB:Q5MNZ6",
  "gene_name": "WD repeat domain phosphoinositide-interacting protein 3",
  "term_id": "GO:0061723",
  "term_label": "glycophagy",
  "gene_symbol": "WDR45B"
}